actin filament organization [GO:0007015] (biological process) Relationships: is a type of supramolecular fiber organization [GO:0097435]; is part of actin cytoskeleton organization [GO:0030036] Definition: A process that is carried out at the cellular level which results in the assembly, arrangement of constituent parts, or disassembly of cytoskeletal structures comprising actin filaments. Includes processes that control the spatial distribution of actin filaments, such as organizing filaments into meshworks, bundles, or other structures, as by cross-linking. Also known as: actin filament organisation, regulation of actin filament localization Sources: GOC:mah Regulation: RO_0002211 by regulation of actin filament organization [GO:0110053] Subtypes: GO:0008154, female germline ring canal formation, actin assembly [GO:0008302], GO:0030240, GO:0045010, actin filament network formation [GO:0051639], actin crosslink formation [GO:0051764], actin filament bundle organization [GO:0061572], GO:0071689, cardiac muscle thin filament assembly [GO:0071691], GO:0090135, actomyosin contractile ring assembly actin filament organization [GO:2000689]